{
  "gene_symbol": "ARRDC1",
  "term_label": "ubiquitin-like ligase-substrate adaptor activity",
  "term_id": "GO:1990756",
  "gene": "UniProtKB:Q8N5I2",
  "gene_name": "Arrestin domain-containing protein 1"
}